{
  "gene_symbol": "CCR4",
  "term_label": "external side of plasma membrane",
  "gene_name": "C-C chemokine receptor type 4",
  "term_id": "GO:0009897",
  "gene": "UniProtKB:P51679"
}